{
  "term_label": "extracellular matrix",
  "gene_symbol": "MATN4",
  "term_id": "GO:0031012",
  "gene": "UniProtKB:O95460",
  "gene_name": "Matrilin-4"
}